{
  "term_id": "GO:0016192",
  "gene_symbol": "CYTH3",
  "gene_name": "Cytohesin-3",
  "term_label": "vesicle-mediated transport",
  "gene": "UniProtKB:O43739"
}